{
  "term_label": "cell-cell adhesion mediated by cadherin",
  "term_id": "GO:0044331",
  "gene": "UniProtKB:Q12864",
  "gene_symbol": "CDH17",
  "gene_name": "Cadherin-17"
}